{
  "gene_name": "Syntaxin-2",
  "term_label": "SNARE complex",
  "gene_symbol": "STX2",
  "term_id": "GO:0031201",
  "gene": "UniProtKB:P32856"
}